positive regulation of response to butan-1-ol [GO:1901450] (biological process) Definition: Any process that activates or increases the frequency, rate or extent of response to butan-1-ol. Sources: GOC:TermGenie, GOC:mengo_curators Relationships: is a type of positive regulation of response to alcohol [GO:1901421]; is a type of GO:1901448; positively regulates response to butan-1-ol [GO:1901422] Also known as: up regulation of response to butan-1-ol, up-regulation of response to butan-1-ol, upregulation of response to butan-1-ol, activation of response to butan-1-ol